alpha-pinene-oxide decyclase activity [GO:0018851] (molecular function) Definition: Catalysis of the reaction: alpha-pinene oxide = (Z)-2-methyl-5-isopropylhexa-2,5-dienal. Sources: EC:5.5.1.10, RHEA:16693 Also known as: alpha-pinene oxide lyase activity, alpha-pinene-oxide lyase (decyclizing) Relationships: is a type of GO:0016872